regulation of histamine secretion by mast cell [GO:1903593] (biological process) References: PMID:18253931 Sources: GOC:TermGenie, GOC:als, GO_REF:0000058 Subtypes: negative regulation of histamine secretion by mast cell [GO:1903594], positive regulation of histamine secretion by mast cell [GO:1903595] Relationships: is a type of regulation of hormone secretion [GO:0046883]; is a type of regulation of inflammatory response [GO:0050727]; is a type of regulation of multicellular organismal process [GO:0051239]; regulates histamine secretion by mast cell [GO:0002553] Definition: Any process that modulates the frequency, rate or extent of histamine secretion by mast cell.